{
  "term_id": "GO:0000139",
  "gene_symbol": "COPG2",
  "gene_name": "Coatomer subunit gamma-2",
  "term_label": "Golgi membrane",
  "gene": "UniProtKB:Q9UBF2"
}